linear element maturation [GO:0062121] (biological process) Definition: The meiotic cell cycle chromosome organization process in which LinE complexes closely associate with chromatin during meiotic prophase to form mature linear elements. Also known as: LinE chromosome loading, LinE focus formation Regulation: regulated by regulation of linear element maturation [GO:0062123] References: PMID:30640914 Relationships: is a type of chromosome organization involved in meiotic cell cycle [GO:0070192]; is part of linear element assembly [GO:0030999]